{
  "term_label": "regulation of centriole replication",
  "gene_name": "Spindle and centriole-associated protein 1",
  "gene": "UniProtKB:Q8N0Z3",
  "term_id": "GO:0046599",
  "gene_symbol": "SPICE1"
}